{
  "gene": "UniProtKB:Q9NS98",
  "term_id": "GO:0038191",
  "term_label": "neuropilin binding",
  "gene_name": "Semaphorin-3G",
  "gene_symbol": "SEMA3G"
}